{
  "gene_symbol": "F11",
  "gene": "UniProtKB:P03951",
  "term_label": "serine-type peptidase activity",
  "term_id": "GO:0008236",
  "gene_name": "Coagulation factor XI"
}